piRNA uni-strand cluster binding [GO:1990471] (molecular function) Definition: Binding to uni-strand piRNA clusters, double-stranded DNA regions that give rise to PIWI-interacting RNAs (piRNAs) that map predominantly to only one strand and exhibit hallmarks of canonical Pol II transcription. Uni-strand piRNA clusters are found in many taxa. References: PMID:24906153 Sources: GOC:bhm Relationships: is a type of piRNA cluster binding [GO:1990470]